{
  "gene_name": "Transmembrane protein 239",
  "term_label": "Unknown molecular function",
  "gene_symbol": "TMEM239",
  "gene": "UniProtKB:Q8WW34",
  "term_id": "UNKNOWN:0001"
}